{
  "gene_name": "Glutamate receptor ionotropic, kainate 5",
  "gene_symbol": "GRIK5",
  "term_label": "presynaptic membrane",
  "term_id": "GO:0042734",
  "gene": "UniProtKB:Q16478"
}